{
  "term_label": "positive regulation of transcription by RNA polymerase II",
  "gene_symbol": "GATA1",
  "term_id": "GO:0045944",
  "gene": "UniProtKB:P15976",
  "gene_name": "Erythroid transcription factor"
}